{
  "gene_name": "C-X-C motif chemokine 17",
  "gene_symbol": "CXCL17",
  "term_id": "GO:0010575",
  "term_label": "positive regulation of vascular endothelial growth factor production",
  "gene": "UniProtKB:Q6UXB2"
}